{
  "gene": "UniProtKB:P40938",
  "term_label": "DNA replication factor C complex",
  "term_id": "GO:0005663",
  "gene_name": "Replication factor C subunit 3",
  "gene_symbol": "RFC3"
}